{
  "gene_symbol": "SCAND1",
  "term_id": "UNKNOWN:0001",
  "term_label": "Unknown molecular function",
  "gene_name": "SCAN domain-containing protein 1",
  "gene": "UniProtKB:P57086"
}